calcium ion export [GO:1901660] (BP) Sources: GOC:TermGenie Definition: The directed movement of calcium ion out of a cell or organelle. Relationships: is a type of GO:0006816